{
  "term_id": "GO:0051879",
  "term_label": "Hsp90 protein binding",
  "gene_name": "Inactive peptidyl-prolyl cis-trans isomerase FKBP6",
  "gene": "UniProtKB:O75344",
  "gene_symbol": "FKBP6"
}